{
  "gene_name": "Phosphatidylinositol 5-phosphate 4-kinase type-2 alpha",
  "gene_symbol": "PIP4K2A",
  "gene": "UniProtKB:P48426",
  "term_label": "phosphatidylinositol phosphate biosynthetic process",
  "term_id": "GO:0046854"
}